{
  "gene_symbol": "KCNS1",
  "term_label": "voltage-gated potassium channel complex",
  "term_id": "GO:0008076",
  "gene_name": "Potassium voltage-gated channel subfamily S member 1",
  "gene": "UniProtKB:Q96KK3"
}